{
  "gene_symbol": "HELT",
  "gene_name": "Hairy and enhancer of split-related protein HELT",
  "gene": "UniProtKB:A6NFD8",
  "term_label": "DNA-binding transcription factor activity, RNA polymerase II-specific",
  "term_id": "GO:0000981"
}